{
  "gene": "UniProtKB:P51684",
  "gene_symbol": "CCR6",
  "gene_name": "C-C chemokine receptor type 6",
  "term_id": "GO:0007204",
  "term_label": "positive regulation of cytosolic calcium ion concentration"
}